Smc5-Smc6 complex [GO:0030915] (cellular component) Definition: A conserved complex that contains a heterodimer of SMC proteins (Smc5p and Smc6p, or homologs thereof) and several other proteins, and is involved in DNA repair and maintaining cell cycle arrest following DNA damage. In S. cerevisiae, this is an octameric complex called Mms21-Smc5-Smc6 complex, with at least five of its subunits conserved in fission yeast and humans. References: PMID:14701739, PMID:15738391, PMID:27373152 Sources: GOC:rb Relationships: is_a SUMO ligase complex [GO:0106068]; is part of GO:0000793